{
  "term_id": "GO:0005634",
  "gene_name": "Cyclin-dependent kinase 2",
  "gene_symbol": "CDK2",
  "term_label": "nucleus",
  "gene": "UniProtKB:P24941"
}